{
  "term_label": "intestine smooth muscle contraction",
  "gene": "UniProtKB:P43115",
  "gene_name": "Prostaglandin E2 receptor EP3 subtype",
  "term_id": "GO:0014827",
  "gene_symbol": "PTGER3"
}